{
  "term_label": "immune response",
  "term_id": "GO:0006955",
  "gene": "UniProtKB:P01624",
  "gene_symbol": "IGKV3-15",
  "gene_name": "Immunoglobulin kappa variable 3-15"
}